{
  "gene": "UniProtKB:Q9BQA5",
  "gene_symbol": "HINFP",
  "term_label": "DNA-binding transcription factor activity, RNA polymerase II-specific",
  "term_id": "GO:0000981",
  "gene_name": "Histone H4 transcription factor"
}